{
  "gene": "UniProtKB:Q49A26",
  "gene_name": "Cytokine-like nuclear factor N-PAC",
  "gene_symbol": "GLYR1",
  "term_id": "GO:0003677",
  "term_label": "DNA binding"
}